{
  "term_id": "GO:0005737",
  "gene_symbol": "LIMS2",
  "gene": "UniProtKB:Q7Z4I7",
  "term_label": "cytoplasm",
  "gene_name": "LIM and senescent cell antigen-like-containing domain protein 2"
}